tectobulbar tract morphogenesis [GO:0034429] (biological process) Definition: Generation of a long process of a CNS neuron, that carries efferent (outgoing) action potentials from the cell body in the optic tectum towards target cells in the premotor reticulospinal system in the hindbrain. References: PMID:15065115, PMID:17507550, PMID:8038988 Sources: GOC:dsf Relationships: is a type of central nervous system projection neuron axonogenesis [GO:0021952]